actin filament-based transport [GO:0099515] (biological process) Subtypes: vesicle transport along actin filament [GO:0030050], nuclear migration along microfilament [GO:0031022], mitochondrion migration along actin filament [GO:0034642] Definition: The transport of organelles or other particles from one location in the cell to another along actin filaments. Sources: GOC:dos, GOC:dph, GOC:mah, GOC:tb Relationships: is a type of GO:0030705